chemokine (C-C motif) ligand 1 production [GO:0071610] (BP) Definition: The appearance of chemokine (C-C motif) ligand 1 due to biosynthesis or secretion following a cellular stimulus, resulting in an increase in its intracellular or extracellular levels. Regulation: regulated by regulation of chemokine (C-C motif) ligand 1 production [GO:0071652]; negatively regulated by negative regulation of chemokine (C-C motif) ligand 1 production [GO:0071653]; positively regulated by positive regulation of chemokine (C-C motif) ligand 1 production [GO:0071654] Sources: GOC:add, GOC:rv Also known as: CCL1 production, T cell activation 3 production, TCA-3 production Relationships: is a type of chemokine production [GO:0032602]